cilium attachment to cell body [GO:0120309] (BP) Definition: A process that is carried out at the cellular level which results in the lateral attachment of the cilium to the cell body via the flagellar attachment zone in some trypanosomatid species. References: PMID:11877446, PMID:18820079, PMID:22623724, PMID:26272611 Sources: GOC:ach, GOC:krc Also known as: cilial attachment to cell body, ciliary attachment to cell body, flagellar attachment to cell body, flagellum attachment to cell body Relationships: is a type of cellular component organization [GO:0016043]; is part of cilium organization [GO:0044782]